{
  "gene_name": "Gasdermin-E",
  "gene_symbol": "GSDME",
  "term_label": "Unknown biological process",
  "gene": "UniProtKB:O60443",
  "term_id": "UNKNOWN:0002"
}